negative regulation of peptide hormone secretion [GO:0090278] (biological process) Subtypes: negative regulation of insulin secretion [GO:0046676], negative regulation of corticotropin secretion [GO:0051460], negative regulation of corticotropin-releasing hormone secretion [GO:0051465], negative regulation of growth hormone secretion [GO:0060125], negative regulation of glucagon secretion [GO:0070093], GO:0090275, negative regulation of prolactin secretion [GO:1902721], negative regulation of calcitonin secretion [GO:1904363], negative regulation of substance P secretion [GO:1904459], negative regulation of thyroid-stimulating hormone secretion [GO:2000613] Sources: GOC:tb Definition: Any process that decreases the rate, frequency, or extent of the regulated release of a peptide hormone from secretory granules. Relationships: is a type of negative regulation of peptide secretion [GO:0002792]; is a type of negative regulation of hormone secretion [GO:0046888]; is a type of regulation of peptide hormone secretion [GO:0090276]; negatively regulates peptide hormone secretion [GO:0030072]